{
  "gene_name": "Protein FAM107B",
  "term_id": "UNKNOWN:0002",
  "gene_symbol": "FAM107B",
  "term_label": "Unknown biological process",
  "gene": "UniProtKB:Q9H098"
}